{
  "gene": "UniProtKB:P41227",
  "term_id": "GO:0031415",
  "gene_name": "N-alpha-acetyltransferase 10",
  "term_label": "NatA complex",
  "gene_symbol": "NAA10"
}